{
  "term_id": "UNKNOWN:0003",
  "term_label": "Unknown cellular component",
  "gene": "UniProtKB:Q8WXX7",
  "gene_symbol": "AUTS2",
  "gene_name": "Autism susceptibility gene 2 protein"
}